{
  "gene_name": "Disintegrin and metalloproteinase domain-containing protein 18",
  "gene": "UniProtKB:Q9Y3Q7",
  "term_id": "GO:0004222",
  "gene_symbol": "ADAM18",
  "term_label": "metalloendopeptidase activity"
}